symbiont-mediated perturbation of host resistance gene-dependent defense response [GO:0052158] (biological process) Definition: Any process in which a symbiont modulates the frequency, rate or extent of the resistance gene-dependent defense response of the host organism. The host is defined as the larger of the organisms involved in a symbiotic interaction. Sources: GOC:mtg_pamgo_17jul06 Also known as: modulation by organism of resistance gene-dependent defense response of other organism involved in symbiotic interaction, modulation by organism of defense response in host by specific elicitors, modulation by organism of host gene-for-gene resistance, modulation by organism of pathogen-race/host plant cultivar-specific resistance in symbiont, modulation by symbiont of host resistance gene-dependent defense response Relationships: is a type of symbiont-mediated perturbation of host defenses [GO:0030682]; is a type of GO:0052167 Subtypes: symbiont-mediated suppression of host resistance gene-dependent defense response [GO:0033660], effector-mediated activation of plant hypersensitive response by symbiont [GO:0080185]